{
  "term_label": "Unknown molecular function",
  "term_id": "UNKNOWN:0001",
  "gene": "UniProtKB:Q8NHX4",
  "gene_name": "Spermatogenesis-associated protein 3",
  "gene_symbol": "SPATA3"
}